{
  "gene_name": "RNA-binding protein MEX3A",
  "term_label": "Unknown biological process",
  "term_id": "UNKNOWN:0002",
  "gene": "UniProtKB:A1L020",
  "gene_symbol": "MEX3A"
}